female germline ring canal inner rim [GO:0035183] (cellular component) Definition: A proteinaceous actin-rich layer of the insect ovarian ring canal that forms subcortically to the outer rim. The electron dense inner rim accumulates after the final mitotic division of each germline syncytia, and contains actin, a phosphotyrosine protein, and a number of cytoskeletal proteins. Relationships: is a type of cellular anatomical structure [GO:0110165]; is part of extracellular region [GO:0005576]; is part of female germline ring canal [GO:0035324] Note: See also the fly_anatomy.ontology term 'inner nurse cell ring canal rim ; FBbt:00004881'. Also known as: germline ring canal inner rim, nurse cell ring canal inner rim, ovarian ring canal inner rim References: PMID:10556087, PMID:7925006, PMID:9093858